{
  "term_id": "GO:0005737",
  "gene": "UniProtKB:P09467",
  "term_label": "cytoplasm",
  "gene_name": "Fructose-1,6-bisphosphatase 1",
  "gene_symbol": "FBP1"
}